high-affinity nickel cation transmembrane transporter activity [GO:0044750] (molecular function) Sources: GOC:jl Definition: Catalysis of the high-affinity transfer of nickel (Ni) cations from one side of a membrane to the other. In high-affinity transport the transporter is able to bind the solute even if it is only present at very low concentrations. Relationships: is a type of nickel cation transmembrane transporter activity [GO:0015099]